{
  "term_label": "neuropeptide signaling pathway",
  "gene_name": "Neurotensin receptor type 2",
  "gene_symbol": "NTSR2",
  "term_id": "GO:0007218",
  "gene": "UniProtKB:O95665"
}